{
  "gene_name": "Polyadenylate-binding protein-interacting protein 1",
  "term_label": "translation activator activity",
  "gene": "UniProtKB:Q9H074",
  "term_id": "GO:0008494",
  "gene_symbol": "PAIP1"
}